{
  "term_label": "Unknown cellular component",
  "gene_symbol": "CT45A10",
  "term_id": "UNKNOWN:0003",
  "gene": "UniProtKB:P0DMU9",
  "gene_name": "Cancer_testis antigen family 45 member A10"
}